{
  "gene": "UniProtKB:P34931",
  "gene_symbol": "HSPA1L",
  "term_label": "nucleus",
  "term_id": "GO:0005634",
  "gene_name": "Heat shock 70 kDa protein 1-like"
}